melibiose transport [GO:0015769] (biological process) Sources: GOC:ai Definition: The directed movement of melibiose into, out of or within a cell, or between cells, by means of some agent such as a transporter or pore. Melibiose is the disaccharide 6-O-alpha-D-galactopyranosyl-D-glucose. Relationships: is a type of disaccharide transport [GO:0015766]